{
  "term_label": "cytoplasmic side of plasma membrane",
  "term_id": "GO:0009898",
  "gene_name": "TNF receptor-associated factor 5",
  "gene": "UniProtKB:O00463",
  "gene_symbol": "TRAF5"
}